basophil degranulation [GO:0002561] (biological process) Regulation: regulated by regulation of basophil degranulation [GO:1903581]; negatively regulated by negative regulation of basophil degranulation [GO:1903582]; positively regulated by positive regulation of basophil degranulation [GO:1903583] Sources: GOC:add, ISBN:0781735149 Relationships: is_a leukocyte degranulation [GO:0043299]; is part of basophil activation involved in immune response [GO:0002276]; is part of GO:0002560 Definition: The regulated exocytosis of secretory granules containing preformed mediators such as histamine, serotonin, and neutral proteases by a basophil.